{
  "term_id": "UNKNOWN:0003",
  "gene": "UniProtKB:P17029",
  "gene_symbol": "ZKSCAN1",
  "term_label": "Unknown cellular component",
  "gene_name": "Zinc finger protein with KRAB and SCAN domains 1"
}